{
  "gene_symbol": "SLC12A6",
  "gene_name": "Solute carrier family 12 member 6",
  "term_label": "chemical synaptic transmission",
  "term_id": "GO:0007268",
  "gene": "UniProtKB:Q9UHW9"
}